{
  "gene_symbol": "SVIP",
  "term_label": "endoplasmic reticulum membrane",
  "term_id": "GO:0005789",
  "gene": "UniProtKB:Q8NHG7",
  "gene_name": "Small VCP_p97-interacting protein"
}